{
  "gene": "UniProtKB:A6NET4",
  "term_id": "GO:0004984",
  "gene_name": "Olfactory receptor 5K3",
  "term_label": "olfactory receptor activity",
  "gene_symbol": "OR5K3"
}